{
  "gene_symbol": "CYFIP1",
  "gene": "UniProtKB:Q7L576",
  "term_id": "GO:0007411",
  "gene_name": "Cytoplasmic FMR1-interacting protein 1",
  "term_label": "axon guidance"
}